{
  "gene_symbol": "FAM86B1",
  "gene_name": "Putative protein N-methyltransferase FAM86B1",
  "term_id": "GO:0032991",
  "term_label": "protein-containing complex",
  "gene": "UniProtKB:Q8N7N1"
}